{
  "term_id": "UNKNOWN:0003",
  "gene": "UniProtKB:Q99576",
  "gene_name": "TSC22 domain family protein 3",
  "gene_symbol": "TSC22D3",
  "term_label": "Unknown cellular component"
}